mast cell activation involved in immune response [GO:0002279] (biological process) Regulation: regulated by regulation of mast cell activation involved in immune response [GO:0033006]; RO_0002212 by negative regulation of mast cell activation involved in immune response [GO:0033007]; positively regulated by GO:0033008 Relationships: is a type of myeloid cell activation involved in immune response [GO:0002275]; is a type of GO:0045576 Definition: The change in morphology and behavior of a mast cell resulting from exposure to a cytokine, chemokine, soluble factor, or to (at least in mammals) an antigen which the mast cell has specifically bound via IgE bound to Fc-epsilonRI receptors, leading to the initiation or perpetuation of an immune response. Also known as: mast cell activation during immune response Sources: GOC:add, ISBN:0781735149